{
  "gene": "UniProtKB:A8MW99",
  "term_label": "spermatogenesis",
  "gene_name": "Meiosis-specific protein MEI4",
  "gene_symbol": "MEI4",
  "term_id": "GO:0007283"
}